{
  "gene_symbol": "KLHL8",
  "gene": "UniProtKB:Q9P2G9",
  "term_label": "cytoplasm",
  "gene_name": "Kelch-like protein 8",
  "term_id": "GO:0005737"
}